{
  "gene": "UniProtKB:Q96JZ2",
  "gene_name": "Hematopoietic SH2 domain-containing protein",
  "gene_symbol": "HSH2D",
  "term_label": "cytoplasm",
  "term_id": "GO:0005737"
}